{
  "term_label": "membrane organization",
  "gene": "UniProtKB:Q9NR31",
  "gene_symbol": "SAR1A",
  "term_id": "GO:0061024",
  "gene_name": "GTP-binding protein SAR1a"
}